{
  "term_label": "chromatin",
  "gene": "UniProtKB:P28749",
  "term_id": "GO:0000785",
  "gene_name": "Retinoblastoma-like protein 1",
  "gene_symbol": "RBL1"
}